{
  "gene_symbol": "CALY",
  "gene_name": "Neuron-specific vesicular protein calcyon",
  "term_label": "endosomal transport",
  "term_id": "GO:0016197",
  "gene": "UniProtKB:Q9NYX4"
}